{
  "gene_name": "Protein Hook homolog 3",
  "gene": "UniProtKB:Q86VS8",
  "term_id": "GO:0008017",
  "gene_symbol": "HOOK3",
  "term_label": "microtubule binding"
}